{
  "gene_symbol": "PREX1",
  "gene": "UniProtKB:Q8TCU6",
  "gene_name": "Phosphatidylinositol 3,4,5-trisphosphate-dependent Rac exchanger 1 protein",
  "term_label": "G protein-coupled receptor signaling pathway",
  "term_id": "GO:0007186"
}